{
  "term_label": "cytoskeleton-dependent intracellular transport",
  "gene_symbol": "MAP6D1",
  "gene": "UniProtKB:Q9H9H5",
  "gene_name": "MAP6 domain-containing protein 1",
  "term_id": "GO:0030705"
}